{
  "term_id": "GO:0005737",
  "gene_name": "Vam6_Vps39-like protein",
  "term_label": "cytoplasm",
  "gene": "UniProtKB:Q96JC1",
  "gene_symbol": "VPS39"
}